chloroplast stroma [GO:0009570] (cellular component) Definition: The space enclosed by the double membrane of a chloroplast but excluding the thylakoid space. It contains DNA, ribosomes and some temporary products of photosynthesis. Relationships: is a type of plastid stroma [GO:0009532]; is part of chloroplast [GO:0009507] Sources: ISBN:0198547684